{
  "gene_name": "UDP-glucose:glycoprotein glucosyltransferase 2",
  "gene": "UniProtKB:Q9NYU1",
  "term_label": "endoplasmic reticulum",
  "term_id": "GO:0005783",
  "gene_symbol": "UGGT2"
}